{
  "term_label": "semaphorin-plexin signaling pathway",
  "gene_symbol": "SEMA3B",
  "gene_name": "Semaphorin-3B",
  "term_id": "GO:0071526",
  "gene": "UniProtKB:Q13214"
}